{
  "gene_symbol": "DNAI3",
  "gene": "UniProtKB:Q8IWG1",
  "term_label": "dynein heavy chain binding",
  "gene_name": "Dynein axonemal intermediate chain 3",
  "term_id": "GO:0045504"
}